{
  "term_id": "UNKNOWN:0001",
  "term_label": "Unknown molecular function",
  "gene": "UniProtKB:Q9BXJ4",
  "gene_name": "Complement C1q tumor necrosis factor-related protein 3",
  "gene_symbol": "C1QTNF3"
}